{
  "gene_name": "Sodium channel protein type 5 subunit alpha",
  "gene": "UniProtKB:Q14524",
  "term_id": "GO:0005248",
  "gene_symbol": "SCN5A",
  "term_label": "voltage-gated sodium channel activity"
}